strombine dehydrogenase activity [GO:0050305] (molecular function) Relationships: is_a oxidoreductase activity, acting on the CH-NH group of donors, NAD or NADP as acceptor [GO:0016646] Definition: Catalysis of the reaction: N-(carboxymethyl)-D-alanine + H2O + NAD+ = glycine + H+ + NADH + pyruvate. Also known as: N-(carboxymethyl)-D-alanine: NAD+ oxidoreductase activity, N-(carboxymethyl)-D-alanine:NAD+ oxidoreductase (glycine-forming), strombine[N-(carboxymethyl)-D-alanine]dehydrogenase activity Sources: EC:1.5.1.22, RHEA:14061